{
  "gene_name": "Non-structural maintenance of chromosomes element 4 homolog A",
  "term_id": "UNKNOWN:0001",
  "gene": "UniProtKB:Q9NXX6",
  "gene_symbol": "NSMCE4A",
  "term_label": "Unknown molecular function"
}